{
  "gene_symbol": "GBGT1",
  "gene_name": "Globoside alpha-1,3-N-acetylgalactosaminyltransferase 1",
  "term_id": "GO:0031982",
  "gene": "UniProtKB:Q8N5D6",
  "term_label": "vesicle"
}